{
  "gene_name": "Rho guanine nucleotide exchange factor TIAM2",
  "gene": "UniProtKB:Q8IVF5",
  "term_id": "GO:0007264",
  "term_label": "small GTPase-mediated signal transduction",
  "gene_symbol": "TIAM2"
}